cardiac conduction system development [GO:0003161] (biological process) Sources: GOC:mtg_heart Relationships: is a type of GO:0048738 Also known as: cardiac impulse conducting system development, heart conduction system development Definition: The process whose specific outcome is the progression of the cardiac conduction system over time, from its formation to the mature structure. The cardiac conduction system consists of specialized cardiomyocytes that regulate the frequency of heart beat.